{
  "gene": "UniProtKB:Q9HBI1",
  "term_id": "GO:0005737",
  "term_label": "cytoplasm",
  "gene_name": "Beta-parvin",
  "gene_symbol": "PARVB"
}